{
  "gene": "UniProtKB:Q15561",
  "gene_symbol": "TEAD4",
  "term_label": "RNA polymerase II cis-regulatory region sequence-specific DNA binding",
  "gene_name": "Transcriptional enhancer factor TEF-3",
  "term_id": "GO:0000978"
}